{
  "term_label": "negative regulation of translation",
  "gene_name": "Protein ZAR1-like",
  "term_id": "GO:0017148",
  "gene_symbol": "ZAR1L",
  "gene": "UniProtKB:A6NP61"
}